D-Ala-D-Ala dipeptidase activity [GO:0160237] (molecular function) Relationships: is a type of dipeptidase activity [GO:0016805] Definition: Catalysis of the reaction: D-alanyl-D-alanine + H2O = 2 D-alanine. References: PMID:7873524 Sources: RHEA:20661 Also known as: D-alanyl-D-alanine dipeptidase activity